{
  "gene_name": "Forkhead box protein O1",
  "gene_symbol": "FOXO1",
  "term_id": "GO:0008286",
  "gene": "UniProtKB:Q12778",
  "term_label": "insulin receptor signaling pathway"
}